{
  "gene_symbol": "FBXO2",
  "gene_name": "F-box only protein 2",
  "term_id": "GO:0036503",
  "term_label": "ERAD pathway",
  "gene": "UniProtKB:Q9UK22"
}